{
  "term_id": "GO:0095500",
  "gene_symbol": "CHRNE",
  "gene_name": "Acetylcholine receptor subunit epsilon",
  "term_label": "acetylcholine receptor signaling pathway",
  "gene": "UniProtKB:Q04844"
}